{
  "term_id": "GO:0006457",
  "gene": "UniProtKB:P50990",
  "term_label": "protein folding",
  "gene_name": "T-complex protein 1 subunit theta",
  "gene_symbol": "CCT8"
}